cilium movement involved in cell motility [GO:0060294] (biological process) Sources: GOC:BHF, GOC:dph, GOC:tb Relationships: is a type of GO:0003341; is part of GO:0060285 Subtypes: GO:0030317 Definition: Movement of cilia mediated by motor proteins that contributes to the movement of a cell. Regulation: regulated by regulation of cilium movement involved in cell motility [GO:0060295]